{
  "term_id": "GO:0035313",
  "gene_name": "Placenta-expressed transcript 1 protein",
  "gene": "UniProtKB:Q6UQ28",
  "gene_symbol": "PLET1",
  "term_label": "wound healing, spreading of epidermal cells"
}